{
  "term_label": "response to oxygen levels",
  "gene_symbol": "GUCY1A1",
  "gene_name": "Guanylate cyclase soluble subunit alpha-1",
  "gene": "UniProtKB:Q02108",
  "term_id": "GO:0070482"
}